androgen secretion [GO:0035935] (biological process) Definition: The regulated release of an androgen into the circulatory system. Androgens are steroid hormones that stimulate or control the development and maintenance of masculine characteristics in vertebrates. Sources: GOC:sl Relationships: is a type of steroid hormone secretion [GO:0035929] Regulation: regulated by regulation of androgen secretion [GO:2000834]; negatively regulated by negative regulation of androgen secretion [GO:2000835]; RO_0002213 by positive regulation of androgen secretion [GO:2000836]